phosphatidylcholine:cardiolipin O-linoleoyltransferase activity [GO:0032577] (molecular function) Also known as: phosphatidylcholine:cardiolipin linoleoyltransferase Definition: Catalysis of the transfer of a linoleoyl ((9Z,12Z)-octadeca-9,12-dienoyl) group from phosphatidylcholine to an oxygen atom on a cardiolipin molecule. Relationships: is_a GO:0032576 Sources: GOC:cb, GOC:mah